{
  "gene": "UniProtKB:Q8N5H3",
  "term_id": "GO:0005737",
  "gene_symbol": "FAM89B",
  "gene_name": "Leucine repeat adapter protein 25",
  "term_label": "cytoplasm"
}